submandibular salivary gland formation [GO:0060661] (biological process) References: PMID:17336109 Sources: GOC:dph Relationships: is a type of anatomical structure formation involved in morphogenesis [GO:0048646]; is part of GO:0007435 Definition: The developmental process pertaining to the initial formation of a submandibular salivary gland. This process begins with a thickening of the epithelium next to the tongue and ends when a bud linked to the oral surface is formed.